E-series resolvin biosynthetic process [GO:0106297] (biological process) Relationships: is a type of GO:0106295 Definition: The chemical reactions and pathways resulting in the formation of resolvin family E-series, hydroxy fatty acids derived from icosapentaenoic acid. References: PMID:21206090